{
  "gene": "UniProtKB:P47804",
  "term_label": "G protein-coupled receptor signaling pathway",
  "term_id": "GO:0007186",
  "gene_symbol": "RGR",
  "gene_name": "RPE-retinal G protein-coupled receptor"
}